{
  "gene_symbol": "TLK1",
  "term_id": "GO:0035556",
  "term_label": "intracellular signal transduction",
  "gene": "UniProtKB:Q9UKI8",
  "gene_name": "Serine_threonine-protein kinase tousled-like 1"
}